{
  "gene_name": "Checkpoint protein HUS1",
  "gene_symbol": "HUS1",
  "gene": "UniProtKB:O60921",
  "term_label": "mitotic DNA replication checkpoint signaling",
  "term_id": "GO:0033314"
}